{
  "term_label": "catenin complex",
  "term_id": "GO:0016342",
  "gene": "UniProtKB:Q13634",
  "gene_symbol": "CDH18",
  "gene_name": "Cadherin-18"
}